negative regulation of sensory perception of pain [GO:1904057] (biological process) References: PMID:17167094 Sources: GOC:TermGenie, GO_REF:0000058 Definition: Any process that stops, prevents or reduces the frequency, rate or extent of sensory perception of pain. Also known as: down regulation of nociception, down regulation of sensory perception of pain, down-regulation of nociception, down-regulation of sensory perception of pain, downregulation of nociception, downregulation of sensory perception of pain, negative regulation of nociception, down regulation of perception of physiological pain, down-regulation of perception of physiological pain, downregulation of perception of physiological pain, inhibition of nociception, inhibition of perception of physiological pain, inhibition of sensory perception of pain, negative regulation of perception of physiological pain Relationships: is a type of negative regulation of nervous system process [GO:0031645]; is a type of regulation of sensory perception of pain [GO:0051930]; negatively regulates sensory perception of pain [GO:0019233]